lipopolysaccharide-mediated signaling pathway [GO:0031663] (biological process) Also known as: LPS-mediated signaling pathway, lipopolysaccharide-mediated signalling pathway Regulation: regulated by regulation of lipopolysaccharide-mediated signaling pathway [GO:0031664]; negatively regulated by negative regulation of lipopolysaccharide-mediated signaling pathway [GO:0031665]; RO_0002213 by positive regulation of lipopolysaccharide-mediated signaling pathway [GO:0031666] Relationships: is a type of GO:0007166; BFO_0000050 GO:0071222 Definition: The series of molecular signals initiated by the binding of a lipopolysaccharide (LPS) to a receptor on the surface of a target cell, and ending with the regulation of a downstream cellular process, e.g. transcription. Lipopolysaccharides are major components of the outer membrane of Gram-negative bacteria, making them prime targets for recognition by the immune system. References: PMID:15379975 Sources: GOC:mah, GOC:signaling